{
  "gene_name": "BTB_POZ domain-containing adapter for CUL3-mediated RhoA degradation protein 3",
  "term_id": "GO:0004842",
  "term_label": "ubiquitin-protein transferase activity",
  "gene": "UniProtKB:Q9H3F6",
  "gene_symbol": "KCTD10"
}